scavenger receptor binding [GO:0005124] (molecular function) Relationships: is a type of signaling receptor binding [GO:0005102] Sources: GOC:ceb Also known as: scavenger receptor ligand Definition: Binding to scavenger receptors, a family of proteins that are expressed on myeloid cells and are involved in the uptake of effete cellular components and foreign particles.